oxidoreductase activity, acting on the CH-CH group of donors, with a flavin as acceptor [GO:0052890] (molecular function) Relationships: is a type of oxidoreductase activity, acting on the CH-CH group of donors [GO:0016627] Subtypes: acyl-CoA dehydrogenase activity [GO:0003995], (R)-benzylsuccinyl-CoA dehydrogenase activity [GO:0033734], 4,4'-diapophytoene desaturase (4,4'-diaponeurosporene-forming) [GO:0102223] Sources: EC:1.3.8.- Definition: Catalysis of an oxidation-reduction (redox) reaction in which a CH-CH group acts as a hydrogen or electron donor and reduces a flavin.